pigment accumulation in tissues [GO:0043480] (biological process) Subtypes: pigment accumulation in tissues in response to UV light [GO:0043479] Relationships: is a type of multicellular organismal process [GO:0032501]; is a type of pigment accumulation [GO:0043476] Sources: GOC:jl Definition: The aggregation of coloring matter in a particular location in a tissue, occurring in response to an external stimulus. Also known as: organismal pigment accumulation